glucuronoarabinoxylan catabolic process [GO:2000887] (biological process) Sources: GOC:mengo_curators Definition: The chemical reactions and pathways resulting in the breakdown of a glucuronoarabinoxylan. Also known as: glucuronoarabinoxylan catabolism Regulation: regulated by regulation of glucuronoarabinoxylan catabolic process [GO:2000918]; negatively regulated by negative regulation of glucuronoarabinoxylan catabolic process [GO:2000919]; positively regulated by positive regulation of glucuronoarabinoxylan catabolic process [GO:2000920] Relationships: is a type of glucuronoxylan catabolic process [GO:2000886]; is_a arabinoxylan-containing compound catabolic process [GO:2000888]